{
  "gene": "UniProtKB:P09110",
  "gene_symbol": "ACAA1",
  "term_label": "fatty acid beta-oxidation",
  "gene_name": "3-ketoacyl-CoA thiolase, peroxisomal",
  "term_id": "GO:0006635"
}